{
  "gene": "UniProtKB:P08195",
  "term_id": "GO:1904273",
  "term_label": "L-alanine import across plasma membrane",
  "gene_name": "4F2 cell-surface antigen heavy chain",
  "gene_symbol": "SLC3A2"
}